{
  "term_label": "unfolded protein binding",
  "gene_symbol": "GRPEL1",
  "gene": "UniProtKB:Q9HAV7",
  "term_id": "GO:0051082",
  "gene_name": "GrpE protein homolog 1, mitochondrial"
}